{
  "gene_symbol": "THSD8",
  "gene_name": "Thrombospondin type-1 domain-containing protein 8",
  "term_label": "Unknown biological process",
  "gene": "UniProtKB:A0A1W2PP97",
  "term_id": "UNKNOWN:0002"
}